{
  "gene": "UniProtKB:Q9UJQ4",
  "gene_name": "Sal-like protein 4",
  "gene_symbol": "SALL4",
  "term_label": "nucleus",
  "term_id": "GO:0005634"
}